curli [GO:0098774] (cellular component) Relationships: is a type of pilus [GO:0009289]; is part of bacterial biofilm matrix [GO:0097311] Definition: A proteinaceous extracellular fiber, produced by an enteric bacterium, that is involved in surface and cell-cell contacts that promote community behavior and host colonization. Also known as: tafi, thin aggregative fimbrae References: PMID:16704339